{
  "term_label": "plasma membrane",
  "gene_name": "Metal transporter CNNM1",
  "term_id": "GO:0005886",
  "gene_symbol": "CNNM1",
  "gene": "UniProtKB:Q9NRU3"
}